transforming growth factor beta receptor superfamily signaling pathway [GO:0141091] (biological process) Definition: The series of molecular signals initiated by an extracellular ligand binding to a member of the transforming growth factor receptor superfamily, and ending with the regulation of a downstream cellular process, e.g. transcription. References: PMID:22651914, PMID:28096268 Also known as: TGF-beta receptor superfamily signaling pathway, TGF-beta receptor superfamily signalling pathway, TGFbeta receptor superfamily signaling pathway, TGFbeta receptor superfamily signalling pathway, transforming growth factor beta receptor superfamily signalling pathway Relationships: is a type of cell surface receptor protein serine/threonine kinase signaling pathway [GO:0007178] Subtypes: GO:0007179, BMP signaling pathway [GO:0030509], activin receptor signaling pathway [GO:0032924]